{
  "term_label": "Unknown biological process",
  "gene": "UniProtKB:Q5T7R7",
  "gene_symbol": "C1orf185",
  "gene_name": "Uncharacterized protein C1orf185",
  "term_id": "UNKNOWN:0002"
}